Cajal-Retzius cell differentiation [GO:0021870] (biological process) Relationships: is a type of cerebral cortex neuron differentiation [GO:0021895] Definition: The process in which a neuroblast acquires specialized structural and/or functional features of a Cajal-Retzius cell, one of a transient population of pioneering neurons in the cerebral cortex. These cells are slender bipolar cells of the developing marginal zone. One feature of these cells in mammals is that they express the Reelin gene. Sources: GOC:cls, GOC:dgh, GOC:dph, GOC:jid, GO_REF:0000021